mismatch base pair DNA N-glycosylase activity [GO:0000700] (molecular function) Relationships: is a type of DNA N-glycosylase activity [GO:0019104] Definition: Catalysis of the removal of single bases present in mismatches by the cleavage the N-C1' glycosidic bond between the target damaged DNA base and the deoxyribose sugar. The reaction releases a free base and leaves an apurinic/apyrimidinic (AP) site. Subtypes: purine-specific mismatch base pair DNA N-glycosylase activity [GO:0000701], pyrimidine-specific mismatch base pair DNA N-glycosylase activity [GO:0008263] References: PMID:9224623 Sources: GOC:elh